{
  "term_id": "GO:0050661",
  "term_label": "NADP binding",
  "gene_name": "Dihydrofolate reductase 2, mitochondrial",
  "gene": "UniProtKB:Q86XF0",
  "gene_symbol": "DHFR2"
}